{
  "term_label": "antimicrobial humoral immune response mediated by antimicrobial peptide",
  "term_id": "GO:0061844",
  "gene": "UniProtKB:Q99877",
  "gene_name": "Histone H2B type 1-N",
  "gene_symbol": "H2BC15"
}